{
  "gene_symbol": "CAT",
  "term_id": "GO:0005737",
  "term_label": "cytoplasm",
  "gene": "UniProtKB:P04040",
  "gene_name": "Catalase"
}